{
  "term_id": "GO:0015878",
  "term_label": "biotin transport",
  "gene": "UniProtKB:Q9Y289",
  "gene_symbol": "SLC5A6",
  "gene_name": "Sodium-dependent multivitamin transporter"
}